{
  "gene_name": "TGF-beta receptor type-1",
  "gene_symbol": "TGFBR1",
  "term_label": "plasma membrane",
  "term_id": "GO:0005886",
  "gene": "UniProtKB:P36897"
}